{
  "gene_symbol": "DDX17",
  "term_id": "GO:1990904",
  "gene": "UniProtKB:Q92841",
  "term_label": "ribonucleoprotein complex",
  "gene_name": "Probable ATP-dependent RNA helicase DDX17"
}